{
  "gene_symbol": "RGS16",
  "term_label": "cytoplasmic side of plasma membrane",
  "gene_name": "Regulator of G-protein signaling 16",
  "gene": "UniProtKB:O15492",
  "term_id": "GO:0009898"
}